{
  "gene": "UniProtKB:P48048",
  "term_id": "UNKNOWN:0001",
  "gene_symbol": "KCNJ1",
  "term_label": "Unknown molecular function",
  "gene_name": "ATP-sensitive inward rectifier potassium channel 1"
}